{
  "gene_name": "F-actin-capping protein subunit alpha-2",
  "term_id": "GO:0051015",
  "gene": "UniProtKB:P47755",
  "term_label": "actin filament binding",
  "gene_symbol": "CAPZA2"
}